{
  "term_label": "pseudouridine synthase activity",
  "gene_name": "H_ACA ribonucleoprotein complex subunit DKC1",
  "gene_symbol": "DKC1",
  "term_id": "GO:0009982",
  "gene": "UniProtKB:O60832"
}